{
  "term_id": "GO:0006974",
  "term_label": "DNA damage response",
  "gene_symbol": "SPRTN",
  "gene": "UniProtKB:Q9H040",
  "gene_name": "DNA-dependent metalloprotease SPRTN"
}